DNA/RNA helicase activity [GO:0033677] (molecular function) Subtypes: 5'-3' DNA/RNA helicase activity [GO:0033678], 3'-5' DNA/RNA helicase activity [GO:0033679] Also known as: ATP-dependent DNA/RNA helicase activity Relationships: is a type of helicase activity [GO:0004386]; is a type of ATP-dependent activity, acting on DNA [GO:0008094]; is a type of ATP-dependent activity, acting on RNA [GO:0008186]; is a type of GO:0140098 Definition: Unwinding of a DNA/RNA duplex, i.e. a double helix in which a strand of DNA pairs with a complementary strand of RNA, driven by ATP hydrolysis. Sources: GOC:mah